lipoyltransferase activity [GO:0017118] (molecular function) Definition: Catalysis of the reaction: (R)-lipoyl-5'-AMP + L-lysyl-[lipoyl-carrier protein] = (R)-N6-lipoyl-L-lysyl-[lipoyl-carrier protein] + AMP + 2 H+. References: PMID:10103005 Sources: RHEA:20473 Relationships: is a type of GO:0016747